{
  "term_label": "epidermal growth factor receptor signaling pathway",
  "term_id": "GO:0007173",
  "gene": "UniProtKB:Q14289",
  "gene_name": "Protein-tyrosine kinase 2-beta",
  "gene_symbol": "PTK2B"
}